{
  "term_id": "UNKNOWN:0001",
  "gene_symbol": "ZNF831",
  "term_label": "Unknown molecular function",
  "gene_name": "Zinc finger protein 831",
  "gene": "UniProtKB:Q5JPB2"
}